{
  "term_label": "nucleus",
  "gene_symbol": "USP17L22",
  "term_id": "GO:0005634",
  "gene_name": "Ubiquitin carboxyl-terminal hydrolase 17-like protein 22",
  "gene": "UniProtKB:D6RA61"
}